{
  "gene_symbol": "RTL10",
  "term_id": "UNKNOWN:0001",
  "gene_name": "Protein Bop",
  "gene": "UniProtKB:Q7L3V2",
  "term_label": "Unknown molecular function"
}